{
  "term_id": "UNKNOWN:0001",
  "term_label": "Unknown molecular function",
  "gene_name": "Placenta-specific gene 8 protein",
  "gene_symbol": "PLAC8",
  "gene": "UniProtKB:Q9NZF1"
}